{
  "term_id": "GO:0031625",
  "gene_symbol": "SPOPL",
  "gene": "UniProtKB:Q6IQ16",
  "gene_name": "Speckle-type POZ protein-like",
  "term_label": "ubiquitin protein ligase binding"
}